{
  "term_label": "Unknown cellular component",
  "gene_name": "Putative uncharacterized protein encoded by COL5A1-AS1",
  "term_id": "UNKNOWN:0003",
  "gene": "UniProtKB:Q5SY13",
  "gene_symbol": "COL5A1-AS1"
}